{
  "gene_symbol": "TTLL9",
  "gene_name": "Probable tubulin polyglutamylase TTLL9",
  "term_id": "GO:0036064",
  "gene": "UniProtKB:Q3SXZ7",
  "term_label": "ciliary basal body"
}